{
  "gene": "UniProtKB:Q8IYX7",
  "term_id": "GO:0036064",
  "gene_symbol": "SAXO1",
  "gene_name": "Stabilizer of axonemal microtubules 1",
  "term_label": "ciliary basal body"
}